protein localization to rhabdomere [GO:1990146] (biological process) References: PMID:8335687 Sources: GOC:sart Definition: A process in which a protein is transported to, or maintained in, a location within a rhabdomere. Relationships: is a type of intracellular protein localization [GO:0008104]